{
  "gene_name": "C-type lectin domain family 2 member A",
  "term_id": "GO:0051132",
  "term_label": "NK T cell activation",
  "gene_symbol": "CLEC2A",
  "gene": "UniProtKB:Q6UVW9"
}